{
  "gene_name": "Putative uncharacterized protein C21orf62-AS1",
  "term_label": "Unknown biological process",
  "gene": "UniProtKB:Q17RA5",
  "term_id": "UNKNOWN:0002",
  "gene_symbol": "C21orf62-AS1"
}